2-hydroxyisoflavanone synthase activity [GO:0033770] (MF) Definition: Catalysis of the reactions: liquiritigenin + O2 + [reduced NADPH--hemoprotein reductase] = 2,4',7-trihydroxyisoflavanone + H2O + [oxidized NADPH--hemoprotein reductase] and (2S)-naringenin + O2 + [reduced NADPH--hemoprotein reductase] = 2,4',5,7-tetrahydroxyisoflavanone + H2O + [oxidized NADPH--hemoprotein reductase]. Relationships: is a type of oxidoreductase activity, acting on paired donors, with incorporation or reduction of molecular oxygen, reduced flavin or flavoprotein as one donor, and incorporation of one atom of oxygen [GO:0016712] Also known as: isoflavonoid synthase Sources: EC:1.14.14.87